{
  "gene_symbol": "TRBV5-5",
  "gene": "UniProtKB:A0A597",
  "term_label": "cell surface receptor signaling pathway",
  "gene_name": "T cell receptor beta variable 5-5",
  "term_id": "GO:0007166"
}